{
  "gene_name": "Ubiquitin-like modifier-activating enzyme 1",
  "term_label": "nucleus",
  "gene": "UniProtKB:P22314",
  "term_id": "GO:0005634",
  "gene_symbol": "UBA1"
}